{
  "term_id": "GO:0030574",
  "term_label": "collagen catabolic process",
  "gene": "UniProtKB:P08253",
  "gene_name": "72 kDa type IV collagenase",
  "gene_symbol": "MMP2"
}